mucosal immune response [GO:0002385] (biological process) Definition: An immune response taking place in mucosal tissues, including those of the intestinal tract, nasal and upper respiratory tract, and genital tract. Relationships: is a type of organ or tissue specific immune response [GO:0002251] Also known as: immune response in MALT, immune response in mucosal-associated lymphoid tissue, immune response in urogenital tract Sources: GOC:jal, GO_REF:0000022, ISBN:0781735149 Subtypes: GO:0002227, mucosal tolerance induction [GO:0002427]